{
  "term_id": "GO:0001750",
  "gene_symbol": "OPN3",
  "gene_name": "Opsin-3",
  "term_label": "photoreceptor outer segment",
  "gene": "UniProtKB:Q9H1Y3"
}